{
  "term_id": "GO:0045198",
  "gene_name": "Nesprin-4",
  "gene": "UniProtKB:Q8N205",
  "gene_symbol": "SYNE4",
  "term_label": "establishment of epithelial cell apical/basal polarity"
}